{
  "gene": "UniProtKB:Q504T8",
  "gene_symbol": "MIDN",
  "term_label": "nucleus",
  "term_id": "GO:0005634",
  "gene_name": "Midnolin"
}